{
  "gene_name": "Protrudin",
  "gene_symbol": "ZFYVE27",
  "gene": "UniProtKB:Q5T4F4",
  "term_id": "GO:0031175",
  "term_label": "neuron projection development"
}